urease activity [GO:0009039] (molecular function) Also known as: urea amidohydrolase activity Regulation: positively regulated by urease activator activity [GO:0018237] Sources: EC:3.5.1.5, RHEA:20557 Definition: Catalysis of the reaction: urea + H2O = CO2 + 2 NH3. Relationships: is a type of hydrolase activity, acting on carbon-nitrogen (but not peptide) bonds, in linear amides [GO:0016811]